{
  "term_id": "GO:0042060",
  "gene_symbol": "EVPL",
  "term_label": "wound healing",
  "gene": "UniProtKB:Q92817",
  "gene_name": "Envoplakin"
}